{
  "term_label": "histone binding",
  "term_id": "GO:0042393",
  "gene_name": "Acidic leucine-rich nuclear phosphoprotein 32 family member A",
  "gene_symbol": "ANP32A",
  "gene": "UniProtKB:P39687"
}